{
  "gene": "UniProtKB:P48444",
  "gene_symbol": "ARCN1",
  "gene_name": "Coatomer subunit delta",
  "term_label": "endoplasmic reticulum to Golgi vesicle-mediated transport",
  "term_id": "GO:0006888"
}